{
  "term_label": "cytosol",
  "gene_name": "Fatty acid-binding protein 5",
  "gene": "UniProtKB:Q01469",
  "term_id": "GO:0005829",
  "gene_symbol": "FABP5"
}